bacterial-type flagellum-dependent swarming motility [GO:0071978] (biological process) Definition: Bacterial-type flagellum-dependent cell motility in which the action of numerous flagella results in the smooth movement of a group of cells along a solid surface. Swarming motility is observed in groups of bacteria. Relationships: is a type of GO:0071973 Also known as: bacterial-type flagellum-mediated cell swarming, bacterial-type flagellar swarming motility References: PMID:14527279, PMID:18461074 Sources: GOC:cilia